{
  "gene": "UniProtKB:P98175",
  "gene_name": "RNA-binding protein 10",
  "gene_symbol": "RBM10",
  "term_label": "nucleus",
  "term_id": "GO:0005634"
}